substrate-bound cell migration, adhesion receptor recycling [GO:0006934] (biological process) References: PMID:11944043 Relationships: is a type of GO:0001881; is part of negative regulation of cell adhesion involved in substrate-bound cell migration [GO:0006933] Definition: The directed movement of accumulated adhesion components such as integrins from the rear of a migrating cell toward the cell front, where they are available to form new protrusions and adhesions.